{
  "term_id": "GO:0042975",
  "term_label": "peroxisome proliferator activated receptor binding",
  "gene_symbol": "ASXL1",
  "gene_name": "Polycomb group protein ASXL1",
  "gene": "UniProtKB:Q8IXJ9"
}